{
  "gene_name": "14-3-3 protein beta_alpha",
  "term_id": "GO:0008104",
  "gene_symbol": "YWHAB",
  "term_label": "intracellular protein localization",
  "gene": "UniProtKB:P31946"
}